mesenchymal cell differentiation involved in renal system development [GO:2001012] (biological process) Subtypes: mesenchymal cell differentiation involved in kidney development [GO:0072161] Relationships: is a type of mesenchymal cell differentiation [GO:0048762]; is part of renal system development [GO:0072001] Definition: The process in which relatively unspecialized cells acquire specialized structural and/or functional features that characterize the mesenchymal cells of the renal system as it progresses from its formation to the mature state. Sources: GOC:mtg_kidney_jan10, GOC:obol, GOC:yaf Also known as: mesenchymal cell differentiation involved in urinary system development, mesenchymal cell differentiation involved in urinary tract development